{
  "gene_symbol": "C1orf43",
  "term_id": "GO:0006909",
  "gene_name": "Protein C1orf43",
  "gene": "UniProtKB:Q9BWL3",
  "term_label": "phagocytosis"
}